{
  "gene": "UniProtKB:Q99715",
  "gene_name": "Collagen alpha-1(XII) chain",
  "term_label": "Unknown cellular component",
  "gene_symbol": "COL12A1",
  "term_id": "UNKNOWN:0003"
}